{
  "term_id": "GO:0016712",
  "gene_symbol": "CYP2J2",
  "gene": "UniProtKB:P51589",
  "gene_name": "Cytochrome P450 2J2",
  "term_label": "oxidoreductase activity, acting on paired donors, with incorporation or reduction of molecular oxygen, reduced flavin or flavoprotein as one donor, and incorporation of one atom of oxygen"
}